{
  "gene": "UniProtKB:A6NDR6",
  "gene_name": "Putative homeobox protein Meis3-like 1",
  "term_id": "GO:0045944",
  "term_label": "positive regulation of transcription by RNA polymerase II",
  "gene_symbol": "MEIS3P1"
}